negative regulation of release of cytochrome c from mitochondria [GO:0090201] (biological process) Sources: GOC:BHF, GOC:dph, GOC:mtg_apoptosis, GOC:tb Note: The release of cytochrome c from mitochondria is a central event in the signaling phase of the apoptotic process, and it is often used by researchers to monitor this type of cell death. Any event that induces apoptosis will at some point induce the release of cytochrome c from mitochondria. Therefore, this term should only be used to annotate gene products that directly and negatively regulate this process. Relationships: is a type of negative regulation of organelle organization [GO:0010639]; is a type of regulation of release of cytochrome c from mitochondria [GO:0090199]; is a type of negative regulation of apoptotic signaling pathway [GO:2001234]; negatively regulates release of cytochrome c from mitochondria [GO:0001836] Definition: Any process that decreases the rate, frequency or extent of release of cytochrome c from mitochondria, the process in which cytochrome c is enabled to move from the mitochondrial intermembrane space into the cytosol, which is an early step in apoptosis and leads to caspase activation.